protein decrotonylase activity [GO:0160008] (molecular function) Definition: Catalysis of the reaction: H2O + N6-(2E)-butenoyl-L-lysyl-[protein] = (2E)-2-butenoate + L-lysyl-[protein]. References: PMID:28497810, PMID:30279482, PMID:34608293 Relationships: is a type of hydrolase activity, acting on carbon-nitrogen (but not peptide) bonds, in linear amides [GO:0016811] Subtypes: histone decrotonylase activity [GO:0160009]